{
  "gene_symbol": "SLIT3",
  "gene": "UniProtKB:O75094",
  "gene_name": "Slit homolog 3 protein",
  "term_label": "Unknown cellular component",
  "term_id": "UNKNOWN:0003"
}